biotin transport [GO:0015878] (biological process) Definition: The directed movement of biotin into, out of or within a cell, or between cells, by means of some agent such as a transporter or pore. Biotin is cis-tetrahydro-2-oxothieno(3,4-d)imidazoline-4-valeric acid; the (+) enantiomer is very widely distributed in cells and serves as a carrier in a number of enzymatic beta-carboxylation reactions. Sources: GOC:ai Also known as: vitamin B7 transport, vitamin H transport Relationships: is a type of monocarboxylic acid transport [GO:0015718]; is a type of GO:0042886; is a type of vitamin transport [GO:0051180]; is a type of sulfur compound transport [GO:0072348] Subtypes: biotin import across plasma membrane [GO:1905135]